{
  "gene_name": "Protein FAM177A1",
  "gene_symbol": "FAM177A1",
  "gene": "UniProtKB:Q8N128",
  "term_id": "UNKNOWN:0002",
  "term_label": "Unknown biological process"
}